{
  "term_id": "GO:0005886",
  "gene": "UniProtKB:Q13574",
  "term_label": "plasma membrane",
  "gene_name": "Diacylglycerol kinase zeta",
  "gene_symbol": "DGKZ"
}